{
  "gene_symbol": "APOBEC3H",
  "gene": "UniProtKB:Q6NTF7",
  "term_label": "cytidine to uridine editing",
  "term_id": "GO:0016554",
  "gene_name": "DNA dC-dU-editing enzyme APOBEC-3H"
}